{
  "term_id": "GO:0040029",
  "gene_name": "Histone deacetylase 4",
  "term_label": "epigenetic regulation of gene expression",
  "gene": "UniProtKB:P56524",
  "gene_symbol": "HDAC4"
}